{
  "gene": "UniProtKB:Q9BU64",
  "term_id": "UNKNOWN:0001",
  "term_label": "Unknown molecular function",
  "gene_symbol": "CENPO",
  "gene_name": "Centromere protein O"
}